{
  "gene": "UniProtKB:O43639",
  "term_label": "cytoplasm",
  "gene_name": "Cytoplasmic protein NCK2",
  "gene_symbol": "NCK2",
  "term_id": "GO:0005737"
}